{
  "gene_name": "Protein TEX261",
  "gene": "UniProtKB:Q6UWH6",
  "term_id": "GO:0005789",
  "gene_symbol": "TEX261",
  "term_label": "endoplasmic reticulum membrane"
}